imaginal disc-derived wing vein morphogenesis [GO:0008586] (BP) Definition: The process in which anatomical structures of the veins on an imaginal disc-derived wing are generated and organized. Sources: GOC:mtg_sensu Relationships: is a type of GO:0009886; is part of GO:0007476 Also known as: wing vein morphogenesis